positive regulation of mitotic cytokinetic process [GO:1903438] (biological process) Subtypes: positive regulation of mitotic division septum assembly [GO:0140281], GO:1903473, positive regulation of mitotic actomyosin contractile ring assembly [GO:1903501], GO:1903617, positive regulation of primary cell septum biogenesis [GO:1905758] Also known as: up regulation of mitotic cytokinetic process, up-regulation of mitotic cytokinetic process, upregulation of mitotic cytokinetic process, activation of mitotic cytokinetic process Sources: GOC:TermGenie, GOC:vw, GO_REF:0000058 Relationships: is a type of regulation of mitotic cytokinetic process [GO:1903436]; is a type of positive regulation of mitotic cytokinesis [GO:1903490]; positively regulates GO:1902410 Definition: Any process that activates or increases the frequency, rate or extent of mitotic cytokinetic process.